assembly of actomyosin apparatus involved in cytokinesis [GO:0000912] (biological process) Definition: The assembly and arrangement of an apparatus composed of actin, myosin, and associated proteins that will function in cytokinesis. Also known as: actomyosin apparatus assembly involved in cytokinesis, cytokinesis, formation of actomyosin apparatus, formation of actomyosin apparatus involved in cytokinesis Relationships: is a type of cellular component assembly [GO:0022607]; is a type of cytokinetic process [GO:0032506]; is part of cytoskeleton-dependent cytokinesis [GO:0061640] Sources: GOC:mtg_cell_cycle Subtypes: GO:0000915, assembly of actomyosin apparatus involved in mitotic cytokinesis [GO:1902407]